{
  "gene_name": "Elongation of very long chain fatty acids protein 5",
  "term_id": "GO:0019367",
  "term_label": "fatty acid elongation, saturated fatty acid",
  "gene": "UniProtKB:Q9NYP7",
  "gene_symbol": "ELOVL5"
}